{
  "gene_symbol": "B4GALT5",
  "gene_name": "Beta-1,4-galactosyltransferase 5",
  "term_label": "UDP-galactose:glucosylceramide beta-1,4-galactosyltransferase activity",
  "gene": "UniProtKB:O43286",
  "term_id": "GO:0008489"
}